presynaptic active zone cytoplasmic component [GO:0098831] (cellular component) Definition: A specialized region below the presynaptic membrane, characterized by electron-dense material, a specialized cytoskeletal matrix and accumulated (associated) synaptic vesicles. Sources: GOC:dos Also known as: cortex of presynaptic active zone, presynaptic zone cortex Relationships: is a type of cell cortex region [GO:0099738]; is part of presynaptic active zone [GO:0048786]